response to L-leucine [GO:0043201] (BP) Definition: Any process that results in a change in state or activity of a cell or an organism (in terms of movement, secretion, enzyme production, gene expression, etc.) as a result of a L-leucine stimulus. Subtypes: cellular response to L-leucine [GO:0071233] Relationships: is a type of response to amino acid [GO:0043200]; is a type of response to nitrogen compound [GO:1901698]; is a type of response to oxygen-containing compound [GO:1901700] Sources: GOC:mlg Also known as: response to leucine